{
  "term_label": "nucleus",
  "gene_symbol": "MAGEC3",
  "gene": "UniProtKB:Q8TD91",
  "gene_name": "Melanoma-associated antigen C3",
  "term_id": "GO:0005634"
}